P-TEFb complex binding [GO:0106140] (molecular function) References: PMID:18391197 Sources: GOC:pga Definition: Binding to a P-TEFb complex. Relationships: is a type of GO:0044877